{
  "gene": "UniProtKB:Q8NGF0",
  "term_label": "plasma membrane",
  "gene_symbol": "OR52B6",
  "term_id": "GO:0005886",
  "gene_name": "Olfactory receptor 52B6"
}